{
  "term_id": "UNKNOWN:0003",
  "gene_name": "TBC1 domain family member 3K",
  "gene": "UniProtKB:A0A087X1G2",
  "gene_symbol": "TBC1D3K",
  "term_label": "Unknown cellular component"
}